{
  "gene": "UniProtKB:Q9UGJ1",
  "term_label": "gamma-tubulin complex",
  "gene_name": "Gamma-tubulin complex component 4",
  "term_id": "GO:0000930",
  "gene_symbol": "TUBGCP4"
}